{
  "gene_symbol": "CLMN",
  "gene": "UniProtKB:Q96JQ2",
  "term_id": "GO:0007097",
  "gene_name": "Calmin",
  "term_label": "nuclear migration"
}